{
  "gene_symbol": "ITIH2",
  "gene": "UniProtKB:P19823",
  "term_label": "Unknown molecular function",
  "gene_name": "Inter-alpha-trypsin inhibitor heavy chain H2",
  "term_id": "UNKNOWN:0001"
}